{
  "gene_symbol": "MARK4",
  "term_id": "GO:0000226",
  "gene_name": "MAP_microtubule affinity-regulating kinase 4",
  "gene": "UniProtKB:Q96L34",
  "term_label": "microtubule cytoskeleton organization"
}